activin binding [GO:0048185] (MF) Sources: GOC:jid, GOC:mah Definition: Binding to activin, a dimer of inhibin-beta subunits. Relationships: is a type of protein-containing complex binding [GO:0044877]